{
  "term_label": "nucleus",
  "gene_symbol": "HSPB6",
  "gene": "UniProtKB:O14558",
  "gene_name": "Heat shock protein beta-6",
  "term_id": "GO:0005634"
}